glucuronide:cation symporter activity [GO:0015488] (molecular function) Sources: TC:2.A.2.3.1 Relationships: is_a GO:0015164; is a type of glycoside-pentoside-hexuronide:cation symporter activity [GO:0015486] Also known as: glucuronide:monovalent cation symporter activity, glucuronoside permease activity Definition: Enables the transfer of a solute or solutes from one side of a membrane to the other according to the reaction: glucuronide(out) + monovalent cation(out) = glucuronide(in) + monovalent cation(in).